{
  "gene_name": "Rho-associated protein kinase 1",
  "term_id": "GO:0000281",
  "gene_symbol": "ROCK1",
  "term_label": "mitotic cytokinesis",
  "gene": "UniProtKB:Q13464"
}